{
  "gene_symbol": "SDCBP",
  "gene_name": "Syntenin-1",
  "gene": "UniProtKB:O00560",
  "term_id": "GO:0030511",
  "term_label": "positive regulation of transforming growth factor beta receptor signaling pathway"
}